{
  "term_id": "GO:0005280",
  "gene_symbol": "SLC36A3",
  "term_label": "amino acid:proton symporter activity",
  "gene": "UniProtKB:Q495N2",
  "gene_name": "Proton-coupled amino acid transporter 3"
}